{
  "term_label": "T cell receptor signaling pathway",
  "gene_symbol": "THEMIS2",
  "gene": "UniProtKB:Q5TEJ8",
  "gene_name": "Protein THEMIS2",
  "term_id": "GO:0050852"
}